{
  "gene_name": "Centrosomal protein of 192 kDa",
  "gene": "UniProtKB:Q8TEP8",
  "term_label": "cytoplasm",
  "gene_symbol": "CEP192",
  "term_id": "GO:0005737"
}